{
  "term_id": "GO:0006357",
  "gene": "UniProtKB:O43345",
  "gene_name": "Zinc finger protein 208",
  "term_label": "regulation of transcription by RNA polymerase II",
  "gene_symbol": "ZNF208"
}